{
  "term_id": "GO:0045053",
  "gene_symbol": "VPS13D",
  "term_label": "protein retention in Golgi apparatus",
  "gene": "UniProtKB:Q5THJ4",
  "gene_name": "Intermembrane lipid transfer protein VPS13D"
}